{
  "gene_name": "Stonin-1",
  "gene": "UniProtKB:Q9Y6Q2",
  "term_id": "GO:0030122",
  "term_label": "AP-2 adaptor complex",
  "gene_symbol": "STON1"
}